{
  "term_id": "GO:0004672",
  "term_label": "protein kinase activity",
  "gene": "UniProtKB:Q59H18",
  "gene_name": "Serine_threonine-protein kinase TNNI3K",
  "gene_symbol": "TNNI3K"
}